{
  "term_label": "protein K63-linked ubiquitination",
  "gene_name": "E3 ubiquitin-protein ligase pellino homolog 3",
  "gene": "UniProtKB:Q8N2H9",
  "gene_symbol": "PELI3",
  "term_id": "GO:0070534"
}